hormone activity [GO:0005179] (molecular function) Relationships: is a type of GO:0048018 Sources: GOC:dph, GOC:mah, ISBN:0198506732 Definition: The action characteristic of a hormone, any substance formed in very small amounts in one specialized organ or group of cells and carried (sometimes in the bloodstream) to another organ or group of cells in the same organism, upon which it has a specific regulatory action. The term was originally applied to agents with a stimulatory physiological action in vertebrate animals (as opposed to a chalone, which has a depressant action). Usage is now extended to regulatory compounds in lower animals and plants, and to synthetic substances having comparable effects; all bind receptors and trigger some biological process. Also known as: cAMP generating peptide activity, glycopeptide hormone, lipopeptide hormone, peptide hormone Subtypes: gonadotropin hormone-releasing hormone activity [GO:0005183], neuropeptide hormone activity [GO:0005184], GO:0008437, diuretic hormone activity [GO:0008613], GO:0016084, GO:0016085, GO:0016521, growth hormone-releasing hormone activity [GO:0016608], follicle-stimulating hormone activity [GO:0016913], melanocyte-stimulating hormone activity [GO:0017044], GO:0017045, melanin-concentrating hormone activity [GO:0030354], GO:0046659, GO:0070186 Note: Also consider annotating to 'receptor agonist activity ; GO:0048018'.